{
  "gene": "UniProtKB:O15146",
  "term_label": "cell surface receptor protein tyrosine kinase signaling pathway",
  "gene_name": "Muscle, skeletal receptor tyrosine-protein kinase",
  "gene_symbol": "MUSK",
  "term_id": "GO:0007169"
}